{
  "term_label": "Unknown biological process",
  "gene_symbol": "FAM153B",
  "gene_name": "Protein FAM153B",
  "term_id": "UNKNOWN:0002",
  "gene": "UniProtKB:P0C7A2"
}